haloperoxidase activity [GO:0140905] (molecular function) References: PMID:28466644, PMID:34368824 Relationships: is a type of peroxidase activity [GO:0004601]; is a type of halogenase activity [GO:0140906] Definition: Catalysis of the reaction: R-CH + a halogen + H2O2 = R-C-halogen + H2O. Subtypes: iodide peroxidase activity [GO:0004447], chloride peroxidase activity [GO:0016691], bromide peroxidase activity [GO:0019806]